{
  "gene": "UniProtKB:P33981",
  "term_label": "meiotic spindle assembly checkpoint signaling",
  "gene_symbol": "TTK",
  "gene_name": "Dual specificity protein kinase TTK",
  "term_id": "GO:0033316"
}